{
  "gene": "UniProtKB:Q3ZM63",
  "term_label": "Unknown biological process",
  "gene_name": "Embryonic testis differentiation protein homolog A",
  "term_id": "UNKNOWN:0002",
  "gene_symbol": "ETDA"
}